{
  "gene_name": "55 kDa erythrocyte membrane protein",
  "gene_symbol": "MPP1",
  "term_label": "signaling receptor binding",
  "gene": "UniProtKB:Q00013",
  "term_id": "GO:0005102"
}